{
  "gene_name": "Neurogenic locus notch homolog protein 1",
  "gene_symbol": "NOTCH1",
  "gene": "UniProtKB:P46531",
  "term_id": "UNKNOWN:0001",
  "term_label": "Unknown molecular function"
}